{
  "term_label": "Cajal body",
  "gene_name": "rRNA 2'-O-methyltransferase fibrillarin",
  "gene": "UniProtKB:P22087",
  "gene_symbol": "FBL",
  "term_id": "GO:0015030"
}